complement component C3a receptor activity [GO:0004876] (MF) Also known as: C3a anaphylatoxin receptor activity Sources: GOC:add, GOC:mah, GOC:pg, GOC:signaling, ISBN:0781735149 Relationships: is a type of GO:0004875 Definition: Combining with the C3a product of the complement cascade and transmitting the signal from one side of the membrane to the other to initiate a change in cell activity.